{
  "gene_symbol": "OLFML2A",
  "gene": "UniProtKB:Q68BL7",
  "term_id": "GO:0005615",
  "term_label": "extracellular space",
  "gene_name": "Olfactomedin-like protein 2A"
}